{
  "term_id": "GO:0030510",
  "term_label": "regulation of BMP signaling pathway",
  "gene_name": "Follistatin-related protein 5",
  "gene": "UniProtKB:Q8N475",
  "gene_symbol": "FSTL5"
}